voltage-gated sodium channel activity involved in cardiac muscle cell action potential [GO:0086006] (MF) Definition: Enables the transmembrane transfer of a sodium ion by a voltage-gated channel through the plasma membrane of a cardiac muscle cell contributing to the depolarization phase of an action potential. A voltage-gated channel is a channel whose open state is dependent on the voltage across the membrane in which it is embedded. Relationships: is a type of voltage-gated sodium channel activity [GO:0005248]; is part of GO:0086012 Sources: GOC:BHF, GOC:mtg_cardiac_conduct_nov11 Subtypes: voltage-gated sodium channel activity involved in AV node cell action potential [GO:0086060], voltage-gated sodium channel activity involved in bundle of His cell action potential [GO:0086061], voltage-gated sodium channel activity involved in Purkinje myocyte action potential [GO:0086062], voltage-gated sodium channel activity involved in SA node cell action potential [GO:0086063]